{
  "gene_symbol": "LMX1A",
  "term_label": "neuron differentiation",
  "gene_name": "LIM homeobox transcription factor 1-alpha",
  "gene": "UniProtKB:Q8TE12",
  "term_id": "GO:0030182"
}